{
  "term_label": "Rap protein signal transduction",
  "gene": "UniProtKB:P10114",
  "gene_symbol": "RAP2A",
  "gene_name": "Ras-related protein Rap-2a",
  "term_id": "GO:0032486"
}